{
  "gene_name": "Interleukin-1 receptor accessory protein",
  "gene_symbol": "IL1RAP",
  "term_id": "GO:0004908",
  "gene": "UniProtKB:Q9NPH3",
  "term_label": "interleukin-1 receptor activity"
}